ascospore wall (1->3)-beta-D-glucan biosynthetic process [GO:0034413] (BP) Relationships: is a type of GO:0034409; is a type of ascospore wall beta-glucan biosynthetic process [GO:0034412]; is a type of fungal-type cell wall (1->3)-beta-D-glucan biosynthetic process [GO:0071970] Regulation: regulated by regulation of ascospore wall (1->3)-beta-D-glucan biosynthetic process [GO:0060624]; positively regulated by positive regulation of regulation of ascospore wall (1->3)-beta-D-glucan biosynthetic process [GO:0140748] Definition: The chemical reactions and pathways resulting in the formation of (1->3)-beta-D-glucans, compounds composed of glucose residues linked by (1->3)-beta-D-glucosidic bonds, found in the walls of ascospores. Also known as: ascospore wall 1,3-beta-D-glucan biosynthetic process, ascospore wall 1,3-beta-glucan biosynthetic process, ascospore wall 1,3-beta-glucan anabolism, ascospore wall 1,3-beta-glucan biosynthesis, ascospore wall 1,3-beta-glucan formation, ascospore wall 1,3-beta-glucan synthesis, ascospore wall beta-1,3-glucan anabolism, ascospore wall beta-1,3-glucan biosynthesis, ascospore wall beta-1,3-glucan biosynthetic process, ascospore wall beta-1,3-glucan formation, ascospore wall beta-1,3-glucan synthesis Sources: GOC:mah